{
  "term_label": "plasma membrane",
  "gene_name": "Cytohesin-1",
  "gene": "UniProtKB:Q15438",
  "gene_symbol": "CYTH1",
  "term_id": "GO:0005886"
}